{
  "gene_name": "Transcriptional regulator QRICH1",
  "gene": "UniProtKB:Q2TAL8",
  "term_label": "Unknown cellular component",
  "gene_symbol": "QRICH1",
  "term_id": "UNKNOWN:0003"
}